amino acid biosynthetic process [GO:0008652] (biological process) Subtypes: GO:0008153, gamma-aminobutyric acid biosynthetic process [GO:0009449], GO:0019483, diaminopimelate biosynthetic process [GO:0019877], nicotianamine biosynthetic process [GO:0030418], GO:0035499, GO:0043102, pyrrolysine biosynthetic process [GO:0071524], GO:1901607 Sources: ISBN:0198506732 Also known as: amino acid anabolism, amino acid biosynthesis, amino acid formation, amino acid synthesis, cellular amino acid biosynthetic process Relationships: is a type of amino acid metabolic process [GO:0006520]; is a type of biosynthetic process [GO:0009058] Definition: The chemical reactions and pathways resulting in the formation of amino acids, organic acids containing one or more amino substituents. Regulation: regulated by regulation of amino acid biosynthetic process [GO:2000282]; negatively regulated by negative regulation of amino acid biosynthetic process [GO:2000283]; RO_0002213 by positive regulation of amino acid biosynthetic process [GO:2000284]